(2R)-oxo-acid reductase activity [GO:0033719] (molecular function) Relationships: is_a oxidoreductase activity, acting on CH-OH group of donors [GO:0016614] Definition: Catalysis of the reaction: a (2R)-hydroxycarboxylate + acceptor = a 2-oxocarboxylate + reduced acceptor. Also known as: 2-oxo-acid reductase activity, (2R)-hydroxy-carboxylate:acceptor oxidoreductase activity, (2R)-hydroxycarboxylate-viologen-oxidoreductase activity, 2-oxoacid reductase activity, HVOR Sources: RHEA:23664 Subtypes: GO:0047809, (2R)-2-hydroxyacid dehydrogenase (NADP+) activity [GO:0050578], (2R)-2-hydroxycarboxylate dehydrogenase activity [GO:0140174], (2R)-hydroxyacid dehydrogenase (quinone) activity [GO:1990464]